FACT complex [GO:0035101] (cellular component) References: PMID:12934006, PMID:12934007, PMID:16678108, PMID:34731638 Relationships: is a type of transcription elongation factor complex [GO:0008023]; is part of chromatin [GO:0000785] Definition: A histone chaperone complex that facilitates nucleosome disassembly and reassembly upon DNA or RNA polymerase passage. Also known as: Facilitates chromatin transcription complex